{
  "gene_symbol": "CNOT3",
  "term_label": "regulation of stem cell population maintenance",
  "term_id": "GO:2000036",
  "gene_name": "CCR4-NOT transcription complex subunit 3",
  "gene": "UniProtKB:O75175"
}